{
  "gene_name": "Atrial natriuretic peptide-converting enzyme",
  "gene_symbol": "CORIN",
  "term_label": "Unknown molecular function",
  "term_id": "UNKNOWN:0001",
  "gene": "UniProtKB:Q9Y5Q5"
}